calcium ion binding involved in regulation of cytosolic calcium ion concentration [GO:0099510] (molecular function) Also known as: regulation of cytosolic calcium ion concentration by calcium ion buffering Relationships: is_a calcium ion binding [GO:0005509]; is part of regulation of cytosolic calcium ion concentration [GO:0051480]; BFO_0000066 GO:0005829 Subtypes: calcium ion binding involved in regulation of presynaptic cytosolic calcium ion concentration [GO:0099534], calcium ion binding involved in regulation of postsynaptic cytosolic calcium ion concentration [GO:0099567] References: PMID:24442513, PMID:26190970 Definition: The directed change of cytosolic calcium ion concentration in the cytosol via the reversible binding of calcium ions to calcium-binding proteins in the cytosol thereby modulating the spatial and temporal dynamics of changes in cytosolic calcium concentrations.